protein-tyrosine sulfotransferase activity [GO:0008476] (molecular function) Definition: Catalysis of the reaction: 3'-phosphoadenosine 5'-phosphosulfate + protein tyrosine = adenosine 3',5'-bisphosphate + protein tyrosine-O-sulfate. Relationships: is a type of sulfotransferase activity [GO:0008146]; is a type of catalytic activity, acting on a protein [GO:0140096] Also known as: protein-tyrosine sulphotransferase activity, 3'-phosphoadenylyl-sulfate:protein-tyrosine O-sulfotransferase activity, tyrosylprotein sulfotransferase activity Sources: EC:2.8.2.20